{
  "term_label": "Unknown molecular function",
  "gene": "UniProtKB:Q96JQ5",
  "gene_symbol": "MS4A4A",
  "term_id": "UNKNOWN:0001",
  "gene_name": "Membrane-spanning 4-domains subfamily A member 4A"
}